{
  "gene_name": "Telomere repeats-binding bouquet formation protein 1",
  "gene": "UniProtKB:Q8NA31",
  "term_label": "Unknown cellular component",
  "gene_symbol": "TERB1",
  "term_id": "UNKNOWN:0003"
}